{
  "gene_name": "Erythropoietin",
  "term_label": "erythropoietin-mediated signaling pathway",
  "term_id": "GO:0038162",
  "gene": "UniProtKB:P01588",
  "gene_symbol": "EPO"
}